{
  "term_label": "TRIF-dependent toll-like receptor signaling pathway",
  "gene_name": "TIR domain-containing adapter molecule 2",
  "term_id": "GO:0035666",
  "gene": "UniProtKB:Q86XR7",
  "gene_symbol": "TICAM2"
}